detection of molecule of fungal origin [GO:0032491] (biological process) Relationships: is a type of GO:0002238; is a type of GO:0009593; is a type of detection of external biotic stimulus [GO:0098581] Also known as: detection of fungal associated molecule, detection of fungus associated molecule Definition: The series of events in which a stimulus from a molecule of fungal origin is received and converted into a molecular signal. Sources: GOC:mah, GOC:rl